{
  "gene_symbol": "TASL",
  "gene": "UniProtKB:Q9HAI6",
  "term_label": "regulation of lysosomal lumen pH",
  "term_id": "GO:0035751",
  "gene_name": "TLR adapter interacting with SLC15A4 on the lysosome"
}